D-ribose metabolic process [GO:0006014] (biological process) Subtypes: D-ribose biosynthetic process [GO:0019302], D-ribose catabolic process [GO:0019303] Sources: ISBN:0198506732 Relationships: is a type of GO:0019321 Definition: The chemical reactions and pathways involving D-ribose (ribo-pentose). As beta-D-ribofuranose, D-ribose forms the glycose group of all ribonucleosides, ribonucleotides and ribonucleic acids, and also of ribose phosphates, various glycosides, some coenzymes and some forms of vitamin B12. Also known as: D-ribose metabolism